{
  "term_id": "GO:0006084",
  "term_label": "acetyl-CoA metabolic process",
  "gene_name": "Hydroxymethylglutaryl-CoA synthase, mitochondrial",
  "gene_symbol": "HMGCS2",
  "gene": "UniProtKB:P54868"
}